{
  "gene_symbol": "RPE65",
  "term_id": "UNKNOWN:0003",
  "term_label": "Unknown cellular component",
  "gene": "UniProtKB:Q16518",
  "gene_name": "Retinoid isomerohydrolase"
}